{
  "term_id": "GO:0000981",
  "gene": "UniProtKB:Q9H8G1",
  "term_label": "DNA-binding transcription factor activity, RNA polymerase II-specific",
  "gene_symbol": "ZNF430",
  "gene_name": "Zinc finger protein 430"
}